{
  "term_id": "UNKNOWN:0002",
  "gene": "UniProtKB:Q9Y399",
  "gene_symbol": "MRPS2",
  "term_label": "Unknown biological process",
  "gene_name": "Small ribosomal subunit protein uS2m"
}